negative regulation of cell growth [GO:0030308] (biological process) Subtypes: negative regulation of axon extension [GO:0030517], negative regulation of collateral sprouting [GO:0048671], negative regulation of sprouting of injured axon [GO:0048688], GO:0051511, GO:0060243, negative regulation of cell growth involved in cardiac muscle cell development [GO:0061052], negative regulation of direction of cell growth [GO:0061391], negative regulation of root hair elongation [GO:1902891], negative regulation of chondrocyte hypertrophy [GO:1903042], negative regulation of dendrite extension [GO:1903860], GO:2000221 Relationships: is a type of GO:0001558; is a type of negative regulation of growth [GO:0045926]; is a type of negative regulation of cellular process [GO:0048523]; negatively regulates cell growth [GO:0016049] Definition: Any process that stops, prevents, or reduces the frequency, rate, extent or direction of cell growth. Also known as: down regulation of cell growth, down-regulation of cell growth, downregulation of cell growth, inhibition of cell growth Sources: GOC:go_curators